{
  "term_id": "UNKNOWN:0003",
  "gene": "UniProtKB:Q11128",
  "term_label": "Unknown cellular component",
  "gene_name": "4-galactosyl-N-acetylglucosaminide 3-alpha-L-fucosyltransferase FUT5",
  "gene_symbol": "FUT5"
}